{
  "gene_symbol": "CELA2B",
  "term_id": "GO:0090330",
  "gene": "UniProtKB:P08218",
  "gene_name": "Chymotrypsin-like elastase family member 2B",
  "term_label": "regulation of platelet aggregation"
}